{
  "gene_symbol": "PIP5K1A",
  "term_label": "1-phosphatidylinositol-4-phosphate 5-kinase activity",
  "term_id": "GO:0016308",
  "gene_name": "Phosphatidylinositol 4-phosphate 5-kinase type-1 alpha",
  "gene": "UniProtKB:Q99755"
}